primary root development [GO:0080022] (biological process) Relationships: is a type of root development [GO:0048364] Definition: The process whose specific outcome is the progression of the primary root over time, from its formation to the mature structure. The primary root develops directly from the embryonic radicle. Sources: GOC:dhl